NADH regeneration [GO:0006735] (biological process) Definition: A metabolic process that generates a pool of NADH by the reduction of NAD+. Relationships: is a type of NAD+ metabolic process [GO:0019674] Sources: GOC:mah Also known as: NAD (reduced) regeneration, reduced NAD regeneration, reduced nicotinamide adenine dinucleotide regeneration